{
  "term_label": "Z disc",
  "gene_name": "Synaptopodin 2-like protein",
  "gene": "UniProtKB:Q9H987",
  "gene_symbol": "SYNPO2L",
  "term_id": "GO:0030018"
}